mycothiol-arsenate ligase activity [GO:0102100] (molecular function) Definition: Catalysis of the reaction: arsenate + mycothiol = mycothiol-arsenate conjugate + H2O. Sources: EC:2.8.4.2, GOC:pz Relationships: is a type of GO:0050497